toluene metabolic process [GO:0018970] (biological process) Definition: The chemical reactions and pathways involving toluene, a volatile monoaromatic hydrocarbon found in crude petroleum and petroleum products such as gasoline and commonly used as a paint thinning agent and in other solvent applications. Sources: GOC:curators Also known as: methylbenzene metabolic process, methylbenzene metabolism, toluene metabolism Relationships: is a type of benzene-containing compound metabolic process [GO:0042537]; is a type of hydrocarbon metabolic process [GO:0120252] Subtypes: toluene oxidation [GO:0019600], toluene catabolic process [GO:0042203], GO:0046252